{
  "gene_symbol": "MAPK3",
  "gene_name": "Mitogen-activated protein kinase 3",
  "term_id": "GO:0007166",
  "gene": "UniProtKB:P27361",
  "term_label": "cell surface receptor signaling pathway"
}